malate-aspartate shuttle [GO:0043490] (biological process) Definition: The process of transferring reducing equivalents from NADH in the cytosol to the mitochondria via malate. Cytosolic aspartate aminotransferase converts aspartate to oxaloacetate, and cytosolic malate dehydrogenase uses NADH to convert oxaloacetate to malate in the cytosol; the malate-alpha-ketoglutarate carrier then transports the malate into the mitochondria where mitochondrial malate dehydrogenase uses NAD to convert malate back to oxaloacetate; the electrons on the reduced NADH are then available for use in the electron transport chain; mitochondrial aspartate aminotransferase converts oxaloacetate to aspartate, and the glutamate-aspartate carrier transports the aspartate back to the cytosol to complete the cycle. Also known as: malate aspartate shuttle, malate/aspartate shuttle, malate:aspartate shuttle Relationships: is a type of NAD+ metabolic process [GO:0019674]; has part GO:0004069; has part L-malate dehydrogenase (NAD+) activity [GO:0030060]; has part mitochondrial transmembrane transport [GO:1990542] References: PMID:16368075 Sources: GOC:sjm